{
  "term_id": "UNKNOWN:0001",
  "gene": "UniProtKB:Q66K66",
  "gene_symbol": "TMEM198",
  "gene_name": "Transmembrane protein 198",
  "term_label": "Unknown molecular function"
}